regulation of glycogen (starch) synthase activity [GO:2000465] (biological process) Subtypes: negative regulation of glycogen (starch) synthase activity [GO:2000466], positive regulation of glycogen (starch) synthase activity [GO:2000467] Definition: Any process that modulates the frequency, rate or extent of glycogen (starch) synthase activity. Relationships: is a type of GO:0051338; regulates GO:0004373 Also known as: regulation of UDP-glucose-glycogen glucosyltransferase activity, regulation of UDP-glucose:glycogen 4-alpha-D-glucosyltransferase activity, regulation of UDP-glycogen synthase activity, regulation of UDPG-glycogen synthetase activity, regulation of UDPG-glycogen transglucosylase activity, regulation of UDPglucose:glycogen 4-alpha-D-glucosyltransferase activity, regulation of glycogen (starch) synthetase activity, regulation of uridine diphosphoglucose-glycogen glucosyltransferase activity Sources: GOC:obol